{
  "term_id": "GO:0021983",
  "term_label": "pituitary gland development",
  "gene_symbol": "HESX1",
  "gene": "UniProtKB:Q9UBX0",
  "gene_name": "Homeobox expressed in ES cells 1"
}